{
  "gene_name": "Urocanate hydratase",
  "gene_symbol": "UROC1",
  "gene": "UniProtKB:Q96N76",
  "term_id": "UNKNOWN:0003",
  "term_label": "Unknown cellular component"
}